{
  "gene_symbol": "NEDD4L",
  "gene_name": "E3 ubiquitin-protein ligase NEDD4-like",
  "term_label": "receptor catabolic process",
  "term_id": "GO:0032801",
  "gene": "UniProtKB:Q96PU5"
}